{
  "term_label": "extracellular matrix structural constituent",
  "term_id": "GO:0005201",
  "gene_symbol": "FBN1",
  "gene": "UniProtKB:P35555",
  "gene_name": "Fibrillin-1"
}